{
  "gene_symbol": "SEMA3D",
  "gene_name": "Semaphorin-3D",
  "term_label": "semaphorin-plexin signaling pathway",
  "term_id": "GO:0071526",
  "gene": "UniProtKB:O95025"
}